{
  "term_id": "UNKNOWN:0001",
  "gene_name": "Tripartite motif-containing protein 66",
  "term_label": "Unknown molecular function",
  "gene": "UniProtKB:O15016",
  "gene_symbol": "TRIM66"
}